{
  "term_label": "G protein-coupled receptor activity",
  "gene_name": "G-protein coupled receptor 39",
  "gene": "UniProtKB:O43194",
  "term_id": "GO:0004930",
  "gene_symbol": "GPR39"
}